{
  "term_id": "GO:0043161",
  "gene": "UniProtKB:P78395",
  "term_label": "proteasome-mediated ubiquitin-dependent protein catabolic process",
  "gene_symbol": "PRAME",
  "gene_name": "Melanoma antigen preferentially expressed in tumors"
}